15-oxoprostaglandin 13-reductase [NAD(P)+] activity [GO:0047522] (molecular function) Relationships: is a type of oxidoreductase activity, acting on the CH-CH group of donors, NAD or NADP as acceptor [GO:0016628] Also known as: (5Z)-(15S)-11alpha-hydroxy-9,15-dioxoprostanoate:NAD(P)+ delta13-oxidoreductase activity, 15-oxo-Delta(13)-prostaglandin reductase activity, 15-oxoprostaglandin 13-oxidase [NAD(P)+] activity, 15-oxoprostaglandin 13-oxidase activity Sources: EC:1.3.1.48 Definition: Catalysis of the reaction: 13,14-dihydro-15-oxo-prostaglandin E2 + NAD(P)+ = 15-oxoprostaglandin E2 + H+ + NAD(P)H.